{
  "gene_symbol": "B3GNT5",
  "term_id": "GO:0016757",
  "gene": "UniProtKB:Q9BYG0",
  "gene_name": "Lactosylceramide 1,3-N-acetyl-beta-D-glucosaminyltransferase",
  "term_label": "glycosyltransferase activity"
}